mitochondrial mRNA surveillance [GO:0035946] (biological process) Definition: The set of processes involved in identifying and degrading messenger RNA (mRNA) within the mitochondrion. Relationships: is a type of mitochondrial mRNA catabolic process [GO:0000958]; is a type of mitochondrial RNA surveillance [GO:2000827] Also known as: mitochondrial aberrant RNA catabolic process, mitochondrial mRNA quality control, mitochondrial messenger RNA surveillance References: PMID:19864255 Sources: GOC:ans